{
  "term_id": "GO:0008821",
  "gene": "UniProtKB:Q9BQ83",
  "term_label": "crossover junction DNA endonuclease activity",
  "gene_symbol": "SLX1A",
  "gene_name": "Structure-specific endonuclease subunit SLX1"
}